{
  "gene_name": "Isthmin-2",
  "term_id": "UNKNOWN:0003",
  "term_label": "Unknown cellular component",
  "gene_symbol": "ISM2",
  "gene": "UniProtKB:Q6H9L7"
}